{
  "gene_symbol": "CES1P1",
  "gene": "UniProtKB:Q9UKY3",
  "term_id": "GO:0005811",
  "gene_name": "Putative inactive carboxylesterase 4",
  "term_label": "lipid droplet"
}